{
  "gene_symbol": "UQCRC2",
  "term_label": "Unknown molecular function",
  "gene_name": "Cytochrome b-c1 complex subunit 2, mitochondrial",
  "gene": "UniProtKB:P22695",
  "term_id": "UNKNOWN:0001"
}